{
  "gene": "UniProtKB:Q13099",
  "gene_name": "Intraflagellar transport protein 88 homolog",
  "term_label": "inner ear receptor cell stereocilium organization",
  "term_id": "GO:0060122",
  "gene_symbol": "IFT88"
}